negative regulation of long-term neuronal synaptic plasticity [GO:0048171] (biological process) References: PMID:11891290 Sources: GOC:jid Also known as: down regulation of long-term neuronal synaptic plasticity, down-regulation of long-term neuronal synaptic plasticity, downregulation of long-term neuronal synaptic plasticity, inhibition of long-term neuronal synaptic plasticity Relationships: is a type of GO:0048169; is a type of GO:0050768 Note: Note that the syntax of the definition of this term is different from the usual regulation syntax because it describes regulation of a trait rather than regulation of a process. Definition: A process that decreases long-term neuronal synaptic plasticity, the ability of neuronal synapses to change long-term as circumstances require. Long-term neuronal synaptic plasticity generally involves increase or decrease in actual synapse numbers.